{
  "term_label": "translation",
  "gene": "UniProtKB:O60783",
  "gene_symbol": "MRPS14",
  "term_id": "GO:0006412",
  "gene_name": "Small ribosomal subunit protein uS14m"
}